{
  "term_label": "DNA-binding transcription repressor activity, RNA polymerase II-specific",
  "gene": "UniProtKB:P24278",
  "term_id": "GO:0001227",
  "gene_symbol": "ZBTB25",
  "gene_name": "Zinc finger and BTB domain-containing protein 25"
}